{
  "term_label": "mammary gland development",
  "gene_symbol": "PRL",
  "gene_name": "Prolactin",
  "gene": "UniProtKB:P01236",
  "term_id": "GO:0030879"
}